{
  "gene_symbol": "KCNJ5-AS1",
  "term_label": "Unknown biological process",
  "gene_name": "Uncharacterized protein KCNJ5-AS1",
  "gene": "UniProtKB:Q8TAV5",
  "term_id": "UNKNOWN:0002"
}